{
  "gene_symbol": "PTH1R",
  "term_id": "GO:0017046",
  "gene_name": "Parathyroid hormone_parathyroid hormone-related peptide receptor",
  "term_label": "peptide hormone binding",
  "gene": "UniProtKB:Q03431"
}